{
  "gene": "UniProtKB:Q96B49",
  "term_label": "Unknown molecular function",
  "gene_symbol": "TOMM6",
  "gene_name": "Mitochondrial import receptor subunit TOM6 homolog",
  "term_id": "UNKNOWN:0001"
}